venom-mediated inhibition of pH-gated ion channel activity [GO:0044735] (biological process) Also known as: envenomation resulting in negative regulation of ASIC channel activity in other organism, envenomation resulting in negative regulation of acid-sensing ion channel activity in another organism, envenomation resulting in negative regulation of acid-sensing ion channel activity in other organism, venom-mediated inhibition of acid-sensing ion channel activity Relationships: is a type of venom-mediated perturbation of pH-gated ion channel activity [GO:0044733] References: PMID:23034652 Sources: GOC:fj, GOC:jl Definition: A process in which an organism inhibits or disrupts the activity of a pH-gated (also known as acid-sensing ion channel (ASIC)) in another organism via the action of a venom.